{
  "gene_symbol": "MEF2A",
  "term_label": "RNA polymerase II cis-regulatory region sequence-specific DNA binding",
  "gene": "UniProtKB:Q02078",
  "term_id": "GO:0000978",
  "gene_name": "Myocyte-specific enhancer factor 2A"
}